{
  "gene_name": "Leucine-rich repeat-containing protein 37A3",
  "gene": "UniProtKB:O60309",
  "term_label": "Unknown molecular function",
  "term_id": "UNKNOWN:0001",
  "gene_symbol": "LRRC37A3"
}